{
  "gene": "UniProtKB:P00492",
  "term_label": "hypoxanthine metabolic process",
  "gene_symbol": "HPRT1",
  "gene_name": "Hypoxanthine-guanine phosphoribosyltransferase",
  "term_id": "GO:0046100"
}